glycerol-phosphate:phosphate antiporter activity [GO:0015527] (molecular function) Sources: TC:2.A.1.4.3 Also known as: glycerol-phosphate:inorganic phosphate antiporter activity Relationships: is a type of GO:0015315; is_a organophosphate ester transmembrane transporter activity [GO:0015605]; is a type of carbohydrate derivative transmembrane transporter activity [GO:1901505] Definition: Enables the transfer of a solute or solutes from one side of a membrane to the other according to the reaction: glycerol phosphate(out) + phosphate(in) = glycerol phosphate(in) + phosphate(out).